{
  "term_id": "GO:0000281",
  "gene_symbol": "ECT2",
  "gene_name": "Protein ECT2",
  "gene": "UniProtKB:Q9H8V3",
  "term_label": "mitotic cytokinesis"
}